{
  "gene_name": "Dickkopf-related protein 3",
  "gene_symbol": "DKK3",
  "term_label": "receptor antagonist activity",
  "gene": "UniProtKB:Q9UBP4",
  "term_id": "GO:0048019"
}